conversion of discoidal high-density lipoprotein particle to spherical high-density lipoprotein particle [GO:0034376] (biological process) Definition: The process in which a discoidal high-density lipoprotein (HDL) particle acquires additional lipid or protein molecules, and cholesterol in the particle is converted to tightly bound cholesterol esters by the action of phosphatidylcholine-sterol O-acyltransferase (lecithin cholesterol acyltransferase; LCAT), resulting in the formation of a spherical HDL particle. Also known as: conversion of discoidal HDL to spherical HDL, discoidal HDL remodeling, discoidal high-density lipoprotein remodeling Sources: GOC:BHF, GOC:mah, GOC:pde Relationships: is a type of GO:0034375